{
  "term_label": "Unknown biological process",
  "gene_name": "Cornifelin",
  "term_id": "UNKNOWN:0002",
  "gene": "UniProtKB:Q9BYD5",
  "gene_symbol": "CNFN"
}